{
  "term_id": "GO:0006869",
  "gene": "UniProtKB:A6NFX1",
  "gene_name": "Sphingosine-1-phosphate transporter MFSD2B",
  "gene_symbol": "MFSD2B",
  "term_label": "lipid transport"
}